{
  "gene_symbol": "MIER2",
  "term_id": "GO:0042826",
  "gene_name": "Mesoderm induction early response protein 2",
  "gene": "UniProtKB:Q8N344",
  "term_label": "histone deacetylase binding"
}